negative regulation of keratinocyte apoptotic process [GO:1902173] (biological process) Relationships: is a type of regulation of keratinocyte apoptotic process [GO:1902172]; is a type of GO:1904036; negatively regulates keratinocyte apoptotic process [GO:0097283] References: PMID:18938133 Sources: GOC:BHF, GOC:TermGenie, GOC:mtg_apoptosis, GOC:rl Also known as: down regulation of keratinocyte apoptotic process, down-regulation of keratinocyte apoptotic process, downregulation of keratinocyte apoptotic process, down regulation of keratinocyte apoptosis, down-regulation of keratinocyte apoptosis, downregulation of keratinocyte apoptosis, inhibition of keratinocyte apoptosis, inhibition of keratinocyte apoptotic process, negative regulation of keratinocyte apoptosis Definition: Any process that stops, prevents or reduces the frequency, rate or extent of keratinocyte apoptotic process.